{
  "gene": "UniProtKB:Q08629",
  "gene_name": "Testican-1",
  "term_label": "regulation of cell-substrate adhesion",
  "gene_symbol": "SPOCK1",
  "term_id": "GO:0010810"
}